{
  "gene_name": "Equilibrative nucleoside transporter 1",
  "term_label": "nucleoside transmembrane transporter activity",
  "term_id": "GO:0005337",
  "gene_symbol": "SLC29A1",
  "gene": "UniProtKB:Q99808"
}